cytoneme morphogenesis [GO:0003399] (BP) Relationships: is a type of GO:0120039 Sources: GOC:ascb_2009, GOC:dph, GOC:tb Definition: The process in which the anatomical structures of a cytoneme are shaped. A cytoneme is a long, thin and polarized actin-based cytoplasmic extension that projects from a cell.